trimethylamine methyltransferase activity [GO:0043834] (molecular function) Definition: Catalysis of the reaction: Co(I)-[trimethylamine-specific corrinoid protein] + H+ + trimethylamine = dimethylamine + methyl-Co(III)-[trimethylamine-specific corrinoid protein]. References: PMID:9006042 Sources: RHEA:39287 Note: This function is the first step in the pathway of methanogenesis from trimethylamine. Also known as: MT1, TMA methyltransferase 1, trimethylamine:corrinoid methyltransferase activity, trimethylamine-specific methylcobalamin:coenzyme M methyltransferase activity, mttB1 Relationships: is a type of methyltransferase activity [GO:0008168]